{
  "term_id": "GO:0007507",
  "gene_name": "Putative teratocarcinoma-derived growth factor 3",
  "term_label": "heart development",
  "gene": "UniProtKB:P51864",
  "gene_symbol": "CRIPTO3"
}